negative regulation of isotype switching to IgG isotypes [GO:0048303] (biological process) Sources: GOC:jid Definition: Any process that stops, prevents, or reduces the frequency, rate or extent of isotype switching to IgG isotypes. Relationships: is a type of negative regulation of isotype switching [GO:0045829]; is a type of regulation of isotype switching to IgG isotypes [GO:0048302]; RO_0002212 isotype switching to IgG isotypes [GO:0048291] Also known as: down regulation of isotype switching to IgG isotypes, down-regulation of isotype switching to IgG isotypes, downregulation of isotype switching to IgG isotypes, negative regulation of class switch recombination to IgG isotypes, negative regulation of class switching to IgG isotypes, negative regulation of isotype switch recombination to IgG isotypes, inhibition of isotype switching to IgG isotypes